{
  "term_label": "cytosol",
  "gene": "UniProtKB:Q16877",
  "term_id": "GO:0005829",
  "gene_name": "6-phosphofructo-2-kinase_fructose-2,6-bisphosphatase 4",
  "gene_symbol": "PFKFB4"
}